{
  "gene": "UniProtKB:Q8N302",
  "gene_symbol": "AGGF1",
  "term_id": "UNKNOWN:0001",
  "gene_name": "Angiogenic factor with G patch and FHA domains 1",
  "term_label": "Unknown molecular function"
}